{
  "gene_symbol": "CADPS2",
  "term_id": "GO:0006887",
  "gene_name": "Calcium-dependent secretion activator 2",
  "gene": "UniProtKB:Q86UW7",
  "term_label": "exocytosis"
}